{
  "term_label": "DNA-binding transcription factor activity, RNA polymerase II-specific",
  "gene": "UniProtKB:Q9NWS9",
  "gene_symbol": "ZNF446",
  "gene_name": "Zinc finger protein 446",
  "term_id": "GO:0000981"
}